positive regulation of secondary cell septum biogenesis [GO:1903397] (biological process) Also known as: up regulation of secondary cell septum biogenesis, up-regulation of secondary cell septum biogenesis, upregulation of secondary cell septum biogenesis, activation of secondary cell septum biogenesis Relationships: is a type of positive regulation of mitotic division septum assembly [GO:0140281]; is a type of GO:1903395; positively regulates secondary cell septum biogenesis [GO:1990344] Definition: Any process that activates or increases the frequency, rate or extent of secondary cell septum biogenesis. References: PMID:23878277 Sources: GOC:TermGenie, GOC:di, GO_REF:0000058